{
  "gene": "UniProtKB:Q5TEU4",
  "gene_name": "Arginine-hydroxylase NDUFAF5, mitochondrial",
  "term_label": "mitochondrion",
  "term_id": "GO:0005739",
  "gene_symbol": "NDUFAF5"
}